{
  "gene": "UniProtKB:Q13443",
  "term_label": "cell-cell adhesion mediated by integrin",
  "gene_name": "Disintegrin and metalloproteinase domain-containing protein 9",
  "gene_symbol": "ADAM9",
  "term_id": "GO:0033631"
}